{
  "term_id": "GO:0120212",
  "gene": "UniProtKB:Q9NWH7",
  "term_label": "sperm head-tail coupling apparatus",
  "gene_name": "Spermatogenesis-associated protein 6",
  "gene_symbol": "SPATA6"
}